{
  "term_label": "Unknown molecular function",
  "gene_symbol": "LTV1",
  "gene": "UniProtKB:Q96GA3",
  "gene_name": "Protein LTV1 homolog",
  "term_id": "UNKNOWN:0001"
}